{
  "term_label": "surfactant homeostasis",
  "gene_symbol": "BPIFA4P",
  "gene_name": "Putative BPIFA4P protein",
  "term_id": "GO:0043129",
  "gene": "UniProtKB:Q86YQ2"
}